{
  "gene_symbol": "CSNK1E",
  "gene": "UniProtKB:P49674",
  "term_label": "signal transduction",
  "term_id": "GO:0007165",
  "gene_name": "Casein kinase I isoform epsilon"
}